{
  "term_id": "GO:0007160",
  "gene_symbol": "FREM1",
  "gene": "UniProtKB:Q5H8C1",
  "gene_name": "FRAS1-related extracellular matrix protein 1",
  "term_label": "cell-matrix adhesion"
}